{
  "term_id": "GO:0006646",
  "term_label": "phosphatidylethanolamine biosynthetic process",
  "gene": "UniProtKB:Q9C0D9",
  "gene_symbol": "SELENOI",
  "gene_name": "Ethanolaminephosphotransferase 1"
}